cellular bud membrane [GO:0033101] (cellular component) Also known as: cellular bud plasma membrane Relationships: is a type of GO:0110165; BFO_0000050 plasma membrane [GO:0005886]; is part of cellular bud [GO:0005933] Sources: GOC:mah Definition: The portion of the plasma membrane surrounding a cellular bud.